{
  "term_id": "GO:0016126",
  "gene_name": "Methylsterol monooxygenase 1",
  "term_label": "sterol biosynthetic process",
  "gene_symbol": "MSMO1",
  "gene": "UniProtKB:Q15800"
}